{
  "term_id": "GO:0005615",
  "gene_name": "Otogelin",
  "gene_symbol": "OTOG",
  "gene": "UniProtKB:Q6ZRI0",
  "term_label": "extracellular space"
}